{
  "gene_name": "Adenomatous polyposis coli protein 2",
  "term_label": "catenin complex",
  "term_id": "GO:0016342",
  "gene_symbol": "APC2",
  "gene": "UniProtKB:O95996"
}